sulfur:ferric ion oxidoreductase activity [GO:0070226] (molecular function) Relationships: is a type of GO:0016667 Definition: Catalysis of the reaction: a perthiol + 4 Fe3+ + 3 H2O = sulfite + a thiol + 4 Fe2+ + 8 H+. Sources: MetaCyc:SULFFEOXIDO-RXN Also known as: hydrogen sulfide:ferric ion oxidoreductase